{
  "gene_name": "Asialoglycoprotein receptor 2",
  "gene": "UniProtKB:P07307",
  "term_id": "GO:0042806",
  "term_label": "fucose binding",
  "gene_symbol": "ASGR2"
}